{
  "term_label": "flagellated sperm motility",
  "gene_symbol": "CATSPER1",
  "term_id": "GO:0030317",
  "gene_name": "Cation channel sperm-associated protein 1",
  "gene": "UniProtKB:Q8NEC5"
}